{
  "gene": "UniProtKB:Q9NV39",
  "term_label": "Unknown cellular component",
  "gene_symbol": "PRR34",
  "gene_name": "Proline-rich protein 34",
  "term_id": "UNKNOWN:0003"
}